{
  "gene_name": "Interleukin-26",
  "term_id": "GO:0006955",
  "gene": "UniProtKB:Q9NPH9",
  "term_label": "immune response",
  "gene_symbol": "IL26"
}